{
  "term_label": "exocytosis",
  "gene_name": "Synaptosomal-associated protein 47",
  "term_id": "GO:0006887",
  "gene_symbol": "SNAP47",
  "gene": "UniProtKB:Q5SQN1"
}